{
  "gene_symbol": "ERV3-1",
  "term_label": "Unknown biological process",
  "gene_name": "Endogenous retrovirus group 3 member 1 Env polyprotein",
  "term_id": "UNKNOWN:0002",
  "gene": "UniProtKB:Q14264"
}